{
  "term_id": "UNKNOWN:0003",
  "gene_name": "F-box only protein 8",
  "gene": "UniProtKB:Q9NRD0",
  "gene_symbol": "FBXO8",
  "term_label": "Unknown cellular component"
}